{
  "gene_symbol": "GIT2",
  "term_label": "synapse",
  "term_id": "GO:0045202",
  "gene_name": "ARF GTPase-activating protein GIT2",
  "gene": "UniProtKB:Q14161"
}